{
  "term_label": "DNA-binding transcription factor activity, RNA polymerase II-specific",
  "gene": "UniProtKB:Q13351",
  "gene_name": "Krueppel-like factor 1",
  "term_id": "GO:0000981",
  "gene_symbol": "KLF1"
}